{
  "gene": "UniProtKB:P19801",
  "term_label": "putrescine metabolic process",
  "gene_symbol": "AOC1",
  "term_id": "GO:0009445",
  "gene_name": "Amiloride-sensitive amine oxidase [copper-containing]"
}